transforming growth factor beta activated kinase 1 complex [GO:0097076] (cellular component) References: PMID:16410796, PMID:17496917, PMID:18021073 Sources: GOC:cna Also known as: TAK1 kinase complex Definition: A protein complex that possesses protein kinase activity and activates the I-kappa B kinase complex (IKK) and mitogen-activated protein (MAP) kinases in response to TRAF6 signaling. It comprises the catalytic subunit TAK1 complexed to the regulatory subunits, termed TABs (TAK1-binding subunits). Relationships: is a type of protein kinase complex [GO:1902911]